{
  "gene_symbol": "CRISP2",
  "gene": "UniProtKB:P16562",
  "term_id": "UNKNOWN:0002",
  "gene_name": "Cysteine-rich secretory protein 2",
  "term_label": "Unknown biological process"
}